{
  "term_label": "Unknown molecular function",
  "gene_symbol": "LNPK",
  "term_id": "UNKNOWN:0001",
  "gene": "UniProtKB:Q9C0E8",
  "gene_name": "Endoplasmic reticulum junction formation protein lunapark"
}